{
  "gene_name": "C-C chemokine receptor-like 2",
  "term_label": "C-C chemokine binding",
  "term_id": "GO:0019957",
  "gene_symbol": "CCRL2",
  "gene": "UniProtKB:O00421"
}